mitochondrial manganese ion transmembrane transport [GO:1990540] (biological process) Relationships: is a type of GO:0071421 References: PMID:12890866 Definition: The process in which a manganese ion is transported across a mitochondrial membrane, into or out of the mitochondrion.